{
  "term_label": "respiratory chain complex I",
  "term_id": "GO:0045271",
  "gene": "UniProtKB:Q16718",
  "gene_name": "NADH dehydrogenase [ubiquinone] 1 alpha subcomplex subunit 5",
  "gene_symbol": "NDUFA5"
}